{
  "term_label": "spermatid development",
  "gene_name": "Testis-specific serine_threonine-protein kinase 2",
  "gene": "UniProtKB:Q96PF2",
  "term_id": "GO:0007286",
  "gene_symbol": "TSSK2"
}